{
  "gene_symbol": "SNX29",
  "term_label": "Unknown molecular function",
  "gene": "UniProtKB:Q8TEQ0",
  "term_id": "UNKNOWN:0001",
  "gene_name": "Sorting nexin-29"
}